{
  "gene": "UniProtKB:P32780",
  "term_label": "transcription factor TFIIH core complex",
  "term_id": "GO:0000439",
  "gene_name": "General transcription factor IIH subunit 1",
  "gene_symbol": "GTF2H1"
}